regulation of protein polyubiquitination [GO:1902914] (BP) Relationships: is a type of regulation of protein ubiquitination [GO:0031396]; regulates protein polyubiquitination [GO:0000209] References: PMID:23645667 Sources: GOC:TermGenie, GOC:di, GO_REF:0000058 Subtypes: regulation of protein K48-linked ubiquitination [GO:0061945], GO:1900044, regulation of protein linear polyubiquitination [GO:1902528], GO:1902915, positive regulation of protein polyubiquitination [GO:1902916] Definition: Any process that modulates the frequency, rate or extent of protein polyubiquitination. Also known as: regulation of protein polyubiquitinylation, regulation of protein polyubiquitylation, regulation of polyubiquitin